{
  "gene_symbol": "KY",
  "term_id": "GO:0007528",
  "gene_name": "Kyphoscoliosis peptidase",
  "term_label": "neuromuscular junction development",
  "gene": "UniProtKB:Q8NBH2"
}